hemocyte proliferation [GO:0035172] (biological process) Sources: GOC:bf, GOC:mtg_sensu Also known as: arthropod blood cell proliferation Definition: The multiplication or reproduction of hemocytes, resulting in the expansion of the cell population. Hemocytes are blood cells associated with a hemocoel (the cavity containing most of the major organs of the arthropod body) which are involved in defense and clotting of hemolymph, but not involved in transport of oxygen. Regulation: regulated by regulation of hemocyte proliferation [GO:0035206]; negatively regulated by negative regulation of hemocyte proliferation [GO:0035207]; RO_0002213 by positive regulation of hemocyte proliferation [GO:0035208] Relationships: is a type of GO:0002376; is a type of cell population proliferation [GO:0008283]